{
  "term_label": "keratinization",
  "term_id": "GO:0031424",
  "gene_name": "Keratin, type II cytoskeletal 6A",
  "gene": "UniProtKB:P02538",
  "gene_symbol": "KRT6A"
}